{
  "gene": "UniProtKB:Q8IW41",
  "term_label": "calcium/calmodulin-dependent protein kinase activity",
  "gene_name": "MAP kinase-activated protein kinase 5",
  "gene_symbol": "MAPKAPK5",
  "term_id": "GO:0004683"
}